threonine deaminase activity [GO:0004794] (molecular function) Also known as: threonine ammonia-lyase activity, threonine dehydratase activity, L-threonine ammonia-lyase (2-oxobutanoate-forming), L-threonine ammonia-lyase activity, L-threonine deaminase activity, L-threonine dehydratase activity, threonine dehydrase activity, L-serine dehydratase activity, L-threonine hydro-lyase (deaminating) activity, serine deaminase activity Sources: EC:4.3.1.19 Definition: Catalysis of the reaction: L-threonine = 2-oxobutanoate + NH4. Relationships: is a type of ammonia-lyase activity [GO:0016841]